{
  "term_id": "GO:0051015",
  "term_label": "actin filament binding",
  "gene": "UniProtKB:P35612",
  "gene_symbol": "ADD2",
  "gene_name": "Beta-adducin"
}